{
  "gene_name": "Protocadherin-8",
  "gene": "UniProtKB:O95206",
  "term_label": "plasma membrane",
  "gene_symbol": "PCDH8",
  "term_id": "GO:0005886"
}